{
  "term_id": "GO:0006355",
  "gene_name": "Zinc finger protein 676",
  "gene": "UniProtKB:Q8N7Q3",
  "term_label": "regulation of DNA-templated transcription",
  "gene_symbol": "ZNF676"
}